{
  "gene_symbol": "PHC3",
  "term_id": "GO:0042393",
  "gene_name": "Polyhomeotic-like protein 3",
  "gene": "UniProtKB:Q8NDX5",
  "term_label": "histone binding"
}